rhamnogalacturonan alpha-L-rhamnopyranosyl-(1->4)-alpha-D-galactopyranosyluronide lyase activity [GO:0046576] (molecular function) References: PMID:8587995, PMID:8720076 Definition: Catalysis of the cleavage of rhamnogalacturonan, generating oligosaccharides of the form alpha-D-us-galacturonic acid-(1,2)-alpha-L-rhamnose-(1,4)-alpha-D-galacturonate-(1,2)-L-rhamnose-(1,2)-alpha-L-rhamnose-p-(1,4)-alpha-D-galacturonic acid, terminating at the non-reducing end with a hex-4-enopyranosyluronic acid residue. Relationships: is a type of GO:0016837 Also known as: rhamnogalacturonase B activity